{
  "gene": "UniProtKB:O14576",
  "gene_name": "Cytoplasmic dynein 1 intermediate chain 1",
  "term_label": "cytoplasmic dynein complex",
  "gene_symbol": "DYNC1I1",
  "term_id": "GO:0005868"
}